{
  "gene": "UniProtKB:Q9Y678",
  "term_id": "GO:0005783",
  "term_label": "endoplasmic reticulum",
  "gene_symbol": "COPG1",
  "gene_name": "Coatomer subunit gamma-1"
}